{
  "gene_symbol": "DANCR",
  "term_label": "Unknown biological process",
  "gene_name": "Putative uncharacterized protein DANCR",
  "term_id": "UNKNOWN:0002",
  "gene": "UniProtKB:P0C864"
}